non-membrane spanning protein tyrosine kinase activity [GO:0004715] (molecular function) Definition: Catalysis of the reaction: ATP + protein L-tyrosine = ADP + protein L-tyrosine phosphate by a non-membrane spanning protein. Sources: EC:2.7.10.2 Relationships: is a type of GO:0004713 Also known as: ATP:protein-tyrosine O-phosphotransferase activity, Bruton's tyrosine kinase activity, cytoplasmic protein tyrosine kinase activity, focal adhesion kinase activity, janus kinase 1 activity, janus kinase 2 activity, janus kinase 3 activity, p60c-src protein tyrosine kinase activity, ATP:protein-L-tyrosine O-phosphotransferase (non-specific) activity, non-specific protein-tyrosine kinase activity